regulation of metaphase plate congression [GO:0090235] (biological process) Definition: Any process that modulates the rate, frequency, or extent of metaphase plate congression, the alignment of chromosomes at the metaphase plate, a plane halfway between the poles of the spindle. Sources: GOC:ascb_2009, GOC:dph, GOC:tb Also known as: regulation of chromosome congression Relationships: is a type of regulation of localization [GO:0032879]; regulates metaphase chromosome alignment [GO:0051310] Subtypes: regulation of attachment of mitotic spindle microtubules to kinetochore [GO:1902423]